{
  "gene": "UniProtKB:P46013",
  "gene_name": "Proliferation marker protein Ki-67",
  "term_id": "GO:0140693",
  "term_label": "molecular condensate scaffold activity",
  "gene_symbol": "MKI67"
}